{
  "gene_symbol": "PREP",
  "term_id": "GO:0070012",
  "gene": "UniProtKB:P48147",
  "term_label": "oligopeptidase activity",
  "gene_name": "Prolyl endopeptidase"
}